{
  "gene_symbol": "RYK",
  "gene_name": "Tyrosine-protein kinase RYK",
  "term_id": "GO:0005886",
  "gene": "UniProtKB:P34925",
  "term_label": "plasma membrane"
}